negative regulation of macrophage colony-stimulating factor signaling pathway [GO:1902227] (biological process) Also known as: down regulation of M-CSF signaling pathway, down regulation of macrophage colony-stimulating factor signaling pathway, down regulation of macrophage colony-stimulating factor signalling pathway, down-regulation of M-CSF signaling pathway, down-regulation of macrophage colony-stimulating factor signaling pathway, down-regulation of macrophage colony-stimulating factor signalling pathway, downregulation of M-CSF signaling pathway, downregulation of macrophage colony-stimulating factor signaling pathway, downregulation of macrophage colony-stimulating factor signalling pathway, negative regulation of M-CSF signaling pathway, negative regulation of macrophage colony-stimulating factor signalling pathway, inhibition of M-CSF signaling pathway, inhibition of macrophage colony-stimulating factor signaling pathway, inhibition of macrophage colony-stimulating factor signalling pathway References: PMID:16705167 Sources: GOC:TermGenie Relationships: is a type of negative regulation of cytokine-mediated signaling pathway [GO:0001960]; is a type of regulation of macrophage colony-stimulating factor signaling pathway [GO:1902226]; negatively regulates macrophage colony-stimulating factor signaling pathway [GO:0038145] Definition: Any process that stops, prevents or reduces the frequency, rate or extent of macrophage colony-stimulating factor signaling pathway.